{
  "gene": "UniProtKB:P48169",
  "term_label": "GABA-A receptor complex",
  "gene_name": "Gamma-aminobutyric acid receptor subunit alpha-4",
  "term_id": "GO:1902711",
  "gene_symbol": "GABRA4"
}